{
  "gene_name": "Hemoglobin subunit beta",
  "gene_symbol": "HBB",
  "gene": "UniProtKB:P68871",
  "term_id": "GO:0020037",
  "term_label": "heme binding"
}